histone H3K4 trimethyltransferase activity [GO:0140999] (molecular function) Note: Comment: Note that the residue position corresponds to the canonical human H3 histone (UniProtKB:P84243); this residue is conserved across all eukaryotes. Residue 1 is the first residue following removal of the initiating Methionine (Met). Note that each histone is encoded by multiple genes, and sequences may vary across different genes within an organism. Also known as: histone H3-K4 trimethylation, histone H3K4 trimethylation, histone H3K4 trimethylase activity, histone lysine N-trimethyltransferase activity (H3-K4 specific) References: PMID:18375658 Sources: RHEA:60260 Relationships: is a type of histone H3K4 methyltransferase activity [GO:0042800] Definition: Catalysis of the reaction: L-lysyl4-[histone H3] + 3 S-adenosyl-L-methionine = 2 H+ + N6,N6-trimethyl-L-lysyl4-[histone H3] + 3 S-adenosyl-L-homocysteine. This reaction is the successive addition of three methyl groups to the unmethylated lysine residue at position 4 of histone H3, producing histone H3K4me3.